{
  "gene_symbol": "SUPT4H1",
  "term_label": "RNA polymerase II complex binding",
  "gene_name": "Transcription elongation factor SPT4",
  "term_id": "GO:0000993",
  "gene": "UniProtKB:P63272"
}